{
  "gene_symbol": "SLC6A8",
  "gene_name": "Sodium- and chloride-dependent creatine transporter 1",
  "term_id": "GO:0035725",
  "term_label": "sodium ion transmembrane transport",
  "gene": "UniProtKB:P48029"
}